{
  "gene_name": "Oxytocin receptor",
  "term_label": "female pregnancy",
  "gene_symbol": "OXTR",
  "term_id": "GO:0007565",
  "gene": "UniProtKB:P30559"
}